{
  "term_label": "negative regulation of transcription by RNA polymerase II",
  "gene": "UniProtKB:P23769",
  "gene_name": "Endothelial transcription factor GATA-2",
  "term_id": "GO:0000122",
  "gene_symbol": "GATA2"
}